establishment of ER localization [GO:0051686] (biological process) Also known as: establishment of ER localisation, establishment of endoplasmic reticulum localization Relationships: is a type of endoplasmic reticulum localization [GO:0051643]; is a type of GO:0051649; is a type of GO:0051656 Subtypes: establishment of endoplasmic reticulum localization to postsynapse [GO:0099089] Sources: GOC:ai Definition: The directed movement of the endoplasmic reticulum to a specific location.